septin ring assembly [GO:0000921] (biological process) Subtypes: GO:0062163 Relationships: is a type of septin ring organization [GO:0031106]; is a type of protein-containing complex assembly [GO:0065003]; is a type of membraneless organelle assembly [GO:0140694] Also known as: septin assembly and septum biosynthesis, septin assembly and septum formation Sources: GOC:clt Definition: The aggregation, arrangement and bonding together of septins and associated proteins to form an organized structure resembling a ring at the cell cortex.